negative regulation by virus of viral protein levels in host cell [GO:0046725] (biological process) Also known as: down regulation of viral protein levels in host cell, down-regulation of viral protein levels in host cell, downregulation of viral protein levels in host cell, negative regulation of viral protein levels, inhibition of viral protein levels in host cell Definition: Any process where the infecting virus reduces the levels of viral proteins in a cell. Sources: GOC:ai Relationships: is a type of GO:0046719; is a type of negative regulation of viral process [GO:0048525]